{
  "gene_name": "Arrestin domain-containing protein 5",
  "gene_symbol": "ARRDC5",
  "term_label": "cytoplasm",
  "term_id": "GO:0005737",
  "gene": "UniProtKB:A6NEK1"
}